{
  "gene_name": "Immunoglobulin lambda joining 3 (Fragment)",
  "gene": "UniProtKB:A0A0A0MT99",
  "term_id": "UNKNOWN:0002",
  "gene_symbol": "IGLJ3",
  "term_label": "Unknown biological process"
}